{
  "term_id": "GO:0005737",
  "term_label": "cytoplasm",
  "gene_name": "Fructose-1,6-bisphosphatase isozyme 2",
  "gene_symbol": "FBP2",
  "gene": "UniProtKB:O00757"
}